{
  "gene_symbol": "USP48",
  "term_id": "GO:0005634",
  "gene": "UniProtKB:Q86UV5",
  "term_label": "nucleus",
  "gene_name": "Ubiquitin carboxyl-terminal hydrolase 48"
}